{
  "gene": "UniProtKB:Q96G30",
  "term_label": "signaling receptor regulator activity",
  "term_id": "GO:0030545",
  "gene_name": "Melanocortin-2 receptor accessory protein 2",
  "gene_symbol": "MRAP2"
}